disaccharide transport [GO:0015766] (biological process) Subtypes: lactose transport [GO:0015767], maltose transport [GO:0015768], melibiose transport [GO:0015769], sucrose transport [GO:0015770], trehalose transport [GO:0015771], GO:0019533, sophorose transport [GO:2001087] Definition: The directed movement of disaccharides into, out of or within a cell, or between cells, by means of some agent such as a transporter or pore. Disaccharides are sugars composed of two monosaccharide units. Sources: GOC:ai Relationships: is_a oligosaccharide transport [GO:0015772]